{
  "gene_name": "Xaa-Pro aminopeptidase 1",
  "term_id": "UNKNOWN:0003",
  "term_label": "Unknown cellular component",
  "gene": "UniProtKB:Q9NQW7",
  "gene_symbol": "XPNPEP1"
}